{
  "gene_symbol": "IMMP2L",
  "gene_name": "Mitochondrial inner membrane protease subunit 2",
  "term_id": "GO:0042720",
  "term_label": "mitochondrial inner membrane peptidase complex",
  "gene": "UniProtKB:Q96T52"
}